{
  "term_id": "GO:0030509",
  "gene_symbol": "TMEM100",
  "gene_name": "Transmembrane protein 100",
  "gene": "UniProtKB:Q9NV29",
  "term_label": "BMP signaling pathway"
}